{
  "term_id": "GO:0007186",
  "gene_name": "Gonadotropin-releasing hormone receptor",
  "term_label": "G protein-coupled receptor signaling pathway",
  "gene": "UniProtKB:P30968",
  "gene_symbol": "GNRHR"
}